{
  "term_label": "nucleosome assembly",
  "gene_symbol": "ATAD2B",
  "gene_name": "ATPase family AAA domain-containing protein 2B",
  "gene": "UniProtKB:Q9ULI0",
  "term_id": "GO:0006334"
}